{
  "gene": "UniProtKB:A8MXY4",
  "term_label": "transcription cis-regulatory region binding",
  "gene_name": "Zinc finger protein 99",
  "gene_symbol": "ZNF99",
  "term_id": "GO:0000976"
}